{
  "gene": "UniProtKB:Q5T7M4",
  "term_label": "negative regulation of gluconeogenesis",
  "gene_name": "Adipolin",
  "term_id": "GO:0045721",
  "gene_symbol": "C1QTNF12"
}